{
  "gene_name": "Small ribosomal subunit protein mS37",
  "gene": "UniProtKB:Q96BP2",
  "gene_symbol": "CHCHD1",
  "term_id": "GO:0005654",
  "term_label": "nucleoplasm"
}